{
  "gene": "UniProtKB:Q96DF8",
  "gene_symbol": "ESS2",
  "term_id": "UNKNOWN:0001",
  "term_label": "Unknown molecular function",
  "gene_name": "Splicing factor ESS-2 homolog"
}